cytolytic granule membrane [GO:0101004] (cellular component) Relationships: is a type of lysosomal membrane [GO:0005765]; is part of cytolytic granule [GO:0044194] References: PMID:17272266, PMID:21247065 Definition: The lipid bilayer surrounding the cytolytic granule.